{
  "gene": "UniProtKB:P68871",
  "gene_symbol": "HBB",
  "term_label": "oxygen transport",
  "term_id": "GO:0015671",
  "gene_name": "Hemoglobin subunit beta"
}